{
  "term_label": "Unknown biological process",
  "term_id": "UNKNOWN:0002",
  "gene_symbol": "MPP3",
  "gene_name": "MAGUK p55 subfamily member 3",
  "gene": "UniProtKB:Q13368"
}